{
  "term_id": "GO:0007420",
  "gene": "UniProtKB:P41225",
  "gene_symbol": "SOX3",
  "gene_name": "Transcription factor SOX-3",
  "term_label": "brain development"
}